carbon fixation [GO:0015977] (biological process) Definition: A metabolic process in which carbon (usually derived from carbon dioxide) is incorporated into organic compounds (usually carbohydrates). Sources: GOC:jl, GOC:mah Also known as: autotrophic CO2 fixation, autotrophic CO2 fixation pathway, autotrophy, carbon dioxide fixation Relationships: is a type of metabolic process [GO:0008152] Subtypes: C4 photosynthesis [GO:0009760], CAM photosynthesis [GO:0009761], GO:0019643, GO:0030634, carbon fixation by 3-hydroxypropionate cycle [GO:0043427]